{
  "term_label": "regulation of Rho protein signal transduction",
  "term_id": "GO:0035023",
  "gene_name": "Rho guanine nucleotide exchange factor 18 (Fragment)",
  "gene": "UniProtKB:A0A590UK10",
  "gene_symbol": "ARHGEF18"
}